{
  "gene_symbol": "GRIA1",
  "term_id": "GO:1904315",
  "gene_name": "Glutamate receptor 1",
  "gene": "UniProtKB:P42261",
  "term_label": "transmitter-gated monoatomic ion channel activity involved in regulation of postsynaptic membrane potential"
}